negative regulation of natural killer cell tolerance induction [GO:0002872] (biological process) Sources: GOC:add Definition: Any process that stops, prevents, or reduces the frequency, rate, or extent of natural killer cell tolerance induction. Relationships: is_a negative regulation of tolerance induction [GO:0002644]; is a type of regulation of acute inflammatory response [GO:0002673]; is a type of regulation of natural killer cell tolerance induction [GO:0002871]; negatively regulates GO:0002519 Also known as: down regulation of natural killer cell tolerance induction, down-regulation of natural killer cell tolerance induction, downregulation of natural killer cell tolerance induction, negative regulation of NK cell tolerance induction, inhibition of natural killer cell tolerance induction